{
  "gene_symbol": "OR5B3",
  "gene": "UniProtKB:Q8NH48",
  "gene_name": "Olfactory receptor 5B3",
  "term_label": "sensory perception of smell",
  "term_id": "GO:0007608"
}